{
  "gene": "UniProtKB:Q8NEN0",
  "gene_name": "Armadillo repeat-containing protein 2",
  "gene_symbol": "ARMC2",
  "term_label": "Unknown cellular component",
  "term_id": "UNKNOWN:0003"
}